{
  "term_label": "GATOR1 complex",
  "gene_symbol": "DEPDC5",
  "gene_name": "GATOR complex protein DEPDC5",
  "gene": "UniProtKB:O75140",
  "term_id": "GO:1990130"
}